{
  "gene": "UniProtKB:Q96A84",
  "term_label": "Unknown cellular component",
  "gene_symbol": "EMID1",
  "term_id": "UNKNOWN:0003",
  "gene_name": "EMI domain-containing protein 1"
}